(3E)-4,8-dimethyl-1,3,7-nonatriene synthase activity [GO:0097008] (molecular function) Definition: Catalysis of the reaction: (E)-nerolidol + NADPH + O2 = (3E)-4,8-dimethylnona-1,3,7-triene + NADP+ + 2 H2O. It is unknown whether this reaction proceeds by the direct release of the 4-carbon compound but-1-en-3-one, or whether the substrate is first degraded to C11-geranylacetone and then cleaved to produce (3E)-4,8-dimethylnona-1,3,7-triene (DMNT) and acetone. Relationships: is a type of oxidoreductase activity, acting on paired donors, with incorporation or reduction of molecular oxygen, NAD(P)H as one donor, and incorporation of one atom of oxygen [GO:0016709] References: PMID:21088219 Sources: GOC:kad, MetaCyc:RXN-8619 Also known as: (3E)-4,8-dimethylnona-1,3,7-triene synthase activity, DNMT synthase activity